{
  "term_label": "endomembrane system",
  "term_id": "GO:0012505",
  "gene_name": "Ras-related protein Rab-24",
  "gene_symbol": "RAB24",
  "gene": "UniProtKB:Q969Q5"
}